endoplasmic reticulum tubular network formation [GO:0071787] (biological process) Relationships: is a type of cellular component assembly [GO:0022607]; is a type of endoplasmic reticulum tubular network organization [GO:0071786] Also known as: ER tubular network assembly, ER tubular network formation, endoplasmic reticulum tubular network assembly Definition: The aggregation, arrangement and bonding together of a set of components to form the endoplasmic reticulum (ER) tubular network. The ER tubular network is the ER part that comprises the membranes with high curvature in cross-section. References: PMID:16469703, PMID:20434336 Sources: GOC:mah, GOC:vw